{
  "gene_symbol": "MAP1S",
  "term_id": "GO:0030425",
  "gene": "UniProtKB:Q66K74",
  "term_label": "dendrite",
  "gene_name": "Microtubule-associated protein 1S"
}